{
  "gene": "UniProtKB:Q6ISB3",
  "term_id": "GO:0005634",
  "gene_symbol": "GRHL2",
  "term_label": "nucleus",
  "gene_name": "Grainyhead-like protein 2 homolog"
}